{
  "gene_name": "Peroxisome proliferator-activated receptor gamma coactivator-related protein 1",
  "term_label": "transcription coactivator activity",
  "gene_symbol": "PPRC1",
  "term_id": "GO:0003713",
  "gene": "UniProtKB:Q5VV67"
}